{
  "term_id": "GO:0031419",
  "gene_name": "Methylmalonyl-CoA mutase, mitochondrial",
  "term_label": "cobalamin binding",
  "gene": "UniProtKB:P22033",
  "gene_symbol": "MMUT"
}